{
  "gene": "UniProtKB:Q9H2S6",
  "term_id": "GO:0001937",
  "term_label": "negative regulation of endothelial cell proliferation",
  "gene_name": "Tenomodulin",
  "gene_symbol": "TNMD"
}